{
  "gene_symbol": "RAP1GAP",
  "term_label": "plasma membrane",
  "term_id": "GO:0005886",
  "gene": "UniProtKB:P47736",
  "gene_name": "Rap1 GTPase-activating protein 1"
}